WD40-repeat domain binding [GO:0071987] (MF) Relationships: is a type of protein domain specific binding [GO:0019904] Also known as: WD domain binding, beta-transducin repeat domain binding Sources: GOC:yaf, InterPro:IPR017986 Definition: Binding to a WD40 repeat domain of a protein. The WD40 repeat is a short structural motif of approximately 40 amino acids, often terminating in a tryptophan-aspartic acid (W-D) dipeptide. Several of these repeats are combined to form a type of protein domain called the WD domain.